{
  "term_id": "GO:0005794",
  "term_label": "Golgi apparatus",
  "gene_symbol": "LARGE1",
  "gene": "UniProtKB:O95461",
  "gene_name": "Xylosyl- and glucuronyltransferase LARGE1"
}